{
  "term_label": "Unknown biological process",
  "gene_name": "Cytochrome P450 4B1",
  "gene_symbol": "CYP4B1",
  "term_id": "UNKNOWN:0002",
  "gene": "UniProtKB:P13584"
}